{
  "term_id": "GO:0000978",
  "gene": "UniProtKB:P26367",
  "gene_symbol": "PAX6",
  "term_label": "RNA polymerase II cis-regulatory region sequence-specific DNA binding",
  "gene_name": "Paired box protein Pax-6"
}